{
  "gene_symbol": "LRRC8A",
  "gene_name": "Volume-regulated anion channel subunit LRRC8A",
  "term_id": "GO:0005225",
  "gene": "UniProtKB:Q8IWT6",
  "term_label": "volume-sensitive anion channel activity"
}